{
  "gene": "UniProtKB:Q15334",
  "gene_symbol": "LLGL1",
  "term_label": "establishment of spindle orientation",
  "gene_name": "Lethal(2) giant larvae protein homolog 1",
  "term_id": "GO:0051294"
}